high-affinity L-arginine transmembrane transporter activity [GO:0005289] (molecular function) Definition: Enables the transfer of arginine from one side of a membrane to the other. In high-affinity transport the transporter is able to bind the solute even if it is only present at very low concentrations. Also known as: high-affinity arginine transporter activity, high affinity arginine transmembrane transporter activity, high-affinity arginine transmembrane transporter activity Sources: GOC:mtg_transport Relationships: is a type of GO:0005287; is a type of L-arginine transmembrane transporter activity [GO:0061459]